{
  "term_id": "GO:0006357",
  "term_label": "regulation of transcription by RNA polymerase II",
  "gene_name": "Zinc finger protein 672",
  "gene_symbol": "ZNF672",
  "gene": "UniProtKB:Q499Z4"
}